{
  "term_id": "GO:0007155",
  "gene_name": "Protocadherin alpha-7",
  "term_label": "cell adhesion",
  "gene_symbol": "PCDHA7",
  "gene": "UniProtKB:Q9UN72"
}